{
  "gene_symbol": "PPP2R2A",
  "term_label": "protein phosphatase regulator activity",
  "gene": "UniProtKB:P63151",
  "gene_name": "Serine_threonine-protein phosphatase 2A 55 kDa regulatory subunit B alpha isoform",
  "term_id": "GO:0019888"
}